arsenate reductase (thioredoxin) activity [GO:0030612] (MF) Sources: RHEA:43848 Relationships: is a type of oxidoreductase activity, acting on phosphorus or arsenic in donors, disulfide as acceptor [GO:0030614] Definition: Catalysis of the reaction: arsenate + [thioredoxin]-dithiol + H+ = arsenite + [thioredoxin]-disulfide + H2O.